{
  "gene_symbol": "MTG2",
  "term_id": "GO:0003924",
  "gene": "UniProtKB:Q9H4K7",
  "term_label": "GTPase activity",
  "gene_name": "Mitochondrial ribosome-associated GTPase 2"
}